histone H3K36me/H3K36me2 demethylase activity [GO:0140680] (molecular function) Relationships: is a type of GO:0051864 Note: Comment: Note that the residue position corresponds to the canonical human H3 histone (UniProtKB:P84243); this residue is conserved across all eukaryotes. Residue 1 is the first residue following removal of the initiating Methionine (Met). Note that each histone is encoded by multiple genes, and sequences may vary across different genes within an organism. Definition: Catalysis of the removal of a methyl group from a di- or a monomethyl-lysine residue at position 36 of the histone H3 protein. This is a dioxygenase reaction that is dependent on Fe(II) and 2-oxoglutarate. Also known as: histone H3K36me2 demethylase activity, histone H3-di/monomethyl-lysine-36 demethylase activity, histone H3K36me demethylase activity References: PMID:20531378